{
  "gene_symbol": "COL6A3",
  "gene": "UniProtKB:P12111",
  "term_id": "UNKNOWN:0003",
  "gene_name": "Collagen alpha-3(VI) chain",
  "term_label": "Unknown cellular component"
}